{
  "gene_symbol": "LMOD3",
  "term_id": "GO:0005865",
  "term_label": "striated muscle thin filament",
  "gene": "UniProtKB:Q0VAK6",
  "gene_name": "Leiomodin-3"
}